{
  "gene_symbol": "LPGAT1",
  "gene": "UniProtKB:Q92604",
  "term_id": "GO:0036149",
  "term_label": "phosphatidylinositol acyl-chain remodeling",
  "gene_name": "Acyl-CoA:lysophosphatidylglycerol acyltransferase 1"
}